negative regulation of response to toluene [GO:1901455] (biological process) Definition: Any process that stops, prevents or reduces the frequency, rate or extent of response to toluene. Sources: GOC:TermGenie, GOC:mengo_curators Also known as: down regulation of response to toluene, down-regulation of response to toluene, downregulation of response to toluene, inhibition of response to toluene Relationships: is a type of negative regulation of response to stimulus [GO:0048585]; is a type of regulation of response to toluene [GO:1901454]; negatively regulates response to toluene [GO:1901424]